{
  "gene": "UniProtKB:Q6T423",
  "gene_symbol": "SLC22A25",
  "term_id": "GO:0015711",
  "term_label": "organic anion transport",
  "gene_name": "Solute carrier family 22 member 25"
}